{
  "gene_name": "Small cysteine and glycine repeat-containing protein 7",
  "term_label": "Unknown molecular function",
  "gene": "UniProtKB:A0A286YF01",
  "term_id": "UNKNOWN:0001",
  "gene_symbol": "SCYGR7"
}